{
  "gene": "UniProtKB:Q9Y614",
  "gene_name": "Actin-like protein 7B",
  "term_label": "Unknown molecular function",
  "term_id": "UNKNOWN:0001",
  "gene_symbol": "ACTL7B"
}